{
  "gene_symbol": "FAM193B",
  "gene_name": "Protein FAM193B",
  "term_label": "cytoplasm",
  "term_id": "GO:0005737",
  "gene": "UniProtKB:Q96PV7"
}